{
  "gene": "UniProtKB:P04629",
  "gene_symbol": "NTRK1",
  "term_label": "nerve growth factor signaling pathway",
  "gene_name": "High affinity nerve growth factor receptor",
  "term_id": "GO:0038180"
}